acetaldehyde metabolic process [GO:0006117] (biological process) Sources: GOC:go_curators Definition: The chemical reactions and pathways involving acetaldehyde, a colorless, flammable liquid intermediate in the metabolism of alcohol. Subtypes: GO:0046186, acetaldehyde catabolic process [GO:0046187] Relationships: is a type of GO:0006081 Also known as: acetaldehyde metabolism, ethanal metabolic process, ethanal metabolism